toll-like receptor TLR1:TLR2 signaling pathway [GO:0038123] (biological process) Relationships: is a type of toll-like receptor signaling pathway [GO:0002224] Definition: The series of molecular signals initiated by a ligand binding of a heterodimeric TLR1:TLR2 complex, followed by transmission of the signal by the activated receptor, and ending with the regulation of a downstream cellular process, e.g. transcription. References: PMID:17318230 Sources: GOC:nhn, GOC:signaling Also known as: TLR2:TLR1 signaling pathway, toll-like receptor TLR1:TLR2 signalling pathway